L-rhamnose 1-dehydrogenase activity [GO:0050034] (molecular function) Also known as: L-rhamnofuranose:NAD+ 1-oxidoreductase activity Definition: Catalysis of the reaction: L-rhamnofuranose + NAD+ = L-rhamnono-1,4-lactone + H+ + NADH. Sources: EC:1.1.1.173, RHEA:12649 Relationships: is a type of oxidoreductase activity, acting on the CH-OH group of donors, NAD or NADP as acceptor [GO:0016616]